symbiont-mediated suppression of host complement activation by inactivation of complement proteins [GO:0141115] (biological process) Also known as: suppression of complement activation by another organism by inactivation of complement proteins Relationships: is a type of symbiont-mediated suppression of host complement activation [GO:0042784] Definition: A process by which a symbiont disrupts or prematurely activates host complement so that its microbial-destroying activities fail. References: PMID:24312361, PMID:34305859